{
  "term_label": "plasma membrane",
  "gene": "UniProtKB:Q7Z410",
  "gene_symbol": "TMPRSS9",
  "term_id": "GO:0005886",
  "gene_name": "Transmembrane protease serine 9"
}